isorhamnetin 3-O-methyltransferase activity [GO:0102444] (molecular function) Sources: RHEA:74759 Definition: Catalysis of the reaction: isorhamnetin + S-adenosyl-L-methionine = 3,3'-O-dimethylquercetin + H+ + S-adenosyl-L-homocysteine. Relationships: is a type of GO:0008168